mitochondrial alpha-ketoglutarate transmembrane transport [GO:1990550] (biological process) Relationships: is a type of alpha-ketoglutarate transport [GO:0015742]; is a type of carboxylic acid transmembrane transport [GO:1905039] References: PMID:11013234, PMID:20371607 Also known as: mitochondrial 2-oxoglutarate transmembrane transport Definition: The process in which alpha-ketoglutarate is transported across a mitochondrial membrane, into or out of the mitochondrion.